{
  "term_id": "UNKNOWN:0003",
  "term_label": "Unknown cellular component",
  "gene_symbol": "CRYBB3",
  "gene_name": "Beta-crystallin B3",
  "gene": "UniProtKB:P26998"
}